{
  "gene_name": "LanC-like protein 3",
  "term_id": "UNKNOWN:0001",
  "gene_symbol": "LANCL3",
  "term_label": "Unknown molecular function",
  "gene": "UniProtKB:Q6ZV70"
}